{
  "term_label": "Unknown cellular component",
  "gene_symbol": "OTUD6A",
  "term_id": "UNKNOWN:0003",
  "gene_name": "OTU domain-containing protein 6A",
  "gene": "UniProtKB:Q7L8S5"
}